{
  "gene_symbol": "CETN1",
  "term_id": "GO:0007099",
  "term_label": "centriole replication",
  "gene_name": "Centrin-1",
  "gene": "UniProtKB:Q12798"
}